{
  "gene_symbol": "CDCA5",
  "term_id": "GO:0000785",
  "gene": "UniProtKB:Q96FF9",
  "gene_name": "Sororin",
  "term_label": "chromatin"
}